{
  "gene": "UniProtKB:Q8N3U4",
  "term_id": "GO:0007062",
  "gene_name": "Cohesin subunit SA-2",
  "term_label": "sister chromatid cohesion",
  "gene_symbol": "STAG2"
}